{
  "term_id": "GO:0060326",
  "term_label": "cell chemotaxis",
  "gene": "UniProtKB:P32302",
  "gene_name": "C-X-C chemokine receptor type 5",
  "gene_symbol": "CXCR5"
}